amino-acid betaine transmembrane transporter activity [GO:0015199] (molecular function) Sources: GOC:ai Also known as: betaine transmembrane transporter activity, betaine/GABA:sodium symporter activity, glycine betaine/proline porter activity, proline/glycine/betaine:hydrogen/sodium symporter activity Subtypes: glycine betaine:proton symporter activity [GO:0015653], ABC-type glycine betaine transporter activity [GO:0031459], glycine betaine:sodium:chloride symporter activity [GO:0140814] Relationships: is a type of quaternary ammonium group transmembrane transporter activity [GO:0015651]; is a type of GO:0072349; is part of GO:0015838 Definition: Enables the transfer of betaine from one side of a membrane to the other. Betaine is the N-trimethyl derivative of an amino acid.